farnesyl diphosphate metabolic process [GO:0045338] (biological process) Also known as: farnesyl diphosphate metabolism Sources: GOC:go_curators Definition: The chemical reactions and pathways involving farnesyl diphosphate, an intermediate in carotenoid, sesquiterpene, squalene and sterol biosynthesis, as well as a substrate in protein farnesylation. Subtypes: GO:0045337, farnesyl diphosphate catabolic process [GO:0045339] Relationships: is a type of GO:0006644; is a type of terpenoid metabolic process [GO:0006721]